arachidonate transport [GO:1903963] (biological process) Definition: The directed movement of an arachidonate into, out of or within a cell, or between cells, by means of some agent such as a transporter or pore. Also known as: arachidonic acid transport Relationships: is a type of long-chain fatty acid transport [GO:0015909]; is a type of icosanoid transport [GO:0071715] Subtypes: arachidonate secretion [GO:0050482] References: PMID:15642721 Sources: GOC:TermGenie, GOC:bhm, GO_REF:0000065